{
  "gene_symbol": "GML",
  "gene": "UniProtKB:Q99445",
  "term_label": "Unknown cellular component",
  "term_id": "UNKNOWN:0003",
  "gene_name": "Glycosyl-phosphatidylinositol-anchored molecule-like protein"
}